{
  "term_label": "Unknown cellular component",
  "gene": "UniProtKB:O75715",
  "gene_name": "Epididymal secretory glutathione peroxidase",
  "gene_symbol": "GPX5",
  "term_id": "UNKNOWN:0003"
}